positive regulation of salivary gland formation by mesenchymal-epithelial signaling [GO:0060639] (biological process) Also known as: positive regulation of salivary gland formation by mesenchymal-epithelial signalling Relationships: is a type of mesenchymal-epithelial cell signaling [GO:0060638]; is a type of positive regulation of animal organ morphogenesis [GO:0110110]; is a type of regulation of multicellular organismal development [GO:2000026]; positively regulates salivary gland morphogenesis [GO:0007435] Sources: GOC:dph Definition: Any process that induces the formation of the salivary gland field by means of the secretion of a signal by a mesenchymal cell and its reception and interpretation by an epithelial cell resulting in it adopting the identity of a salivary gland bud cell.